{
  "term_label": "fibroblast growth factor receptor signaling pathway",
  "gene_symbol": "CHURC1",
  "term_id": "GO:0008543",
  "gene_name": "Protein Churchill",
  "gene": "UniProtKB:Q8WUH1"
}